mammary gland morphogenesis [GO:0060443] (biological process) Sources: GOC:dph Definition: The process in which anatomical structures of the mammary gland are generated and organized. Morphogenesis refers to the creation of shape. The mammary gland is a large compound sebaceous gland that in female mammals is modified to secrete milk. Relationships: is a type of gland morphogenesis [GO:0022612]; is part of GO:0030879